extrasynaptic signaling via GABA [GO:0160001] (biological process) References: PMID:23038269, PMID:9364051 Definition: Cell-cell signaling that starts with the activation of extrasynaptic GABA receptors in neurons through binding of ambient gamma-aminobutyric acid present in the extracellular fluid. Relationships: is_a GO:0007214